{
  "gene_symbol": "ZNF90",
  "gene_name": "Zinc finger protein 90",
  "term_id": "UNKNOWN:0003",
  "gene": "UniProtKB:Q03938",
  "term_label": "Unknown cellular component"
}